U11/U12 snRNP [GO:0034693] (cellular component) Definition: A ribonucleoprotein complex that is formed by the association of the U11 and U12 small nuclear ribonucleoproteins. References: PMID:15146077 Sources: GOC:mah Also known as: snRNP U11/U12, 18S U11/U12 snRNP Relationships: is a type of spliceosomal snRNP complex [GO:0097525]